maintenance of protein localization at cell tip [GO:0099017] (biological process) Subtypes: GO:0099019 Relationships: is_a GO:0032507; occurs in cell tip [GO:0051286] Also known as: maintenance of protein location at cell tip Definition: Any process in which localization of a protein is maintained at the cell tip. References: PMID:12894167 Sources: GOC:dos, GOC:vw